L-histidine catabolic process to imidazol-5-yl-lactate [GO:0019559] (BP) Definition: The chemical reactions and pathways resulting in the breakdown of L-histidine into other compounds, including imidazol-5-yl-lactate. Sources: GOC:go_curators Also known as: histidine breakdown to imidazol-5-yl-lactate, histidine degradation to imidazol-5-yl-lactate Relationships: is a type of GO:0006548